sodium-dependent phosphate transport [GO:0044341] (biological process) Definition: The directed movement of phosphate into, out of or within a cell, or between cells, by means of some agent such as a transporter or pore, by a mechanism dependent upon sodium ions. Regulation: regulated by regulation of sodium-dependent phosphate transport [GO:2000118]; negatively regulated by negative regulation of sodium-dependent phosphate transport [GO:2000119]; positively regulated by positive regulation of sodium-dependent phosphate transport [GO:2000120] Sources: GOC:BHF, GOC:jl Relationships: is a type of phosphate ion transport [GO:0006817]